{
  "term_id": "GO:0005102",
  "gene_symbol": "NXPH2",
  "term_label": "signaling receptor binding",
  "gene_name": "Neurexophilin-2",
  "gene": "UniProtKB:O95156"
}